{
  "term_id": "GO:0010774",
  "gene": "UniProtKB:Q9P2W1",
  "gene_name": "Homologous-pairing protein 2 homolog",
  "gene_symbol": "PSMC3IP",
  "term_label": "meiotic strand invasion involved in reciprocal meiotic recombination"
}